{
  "gene_name": "Bile acid-CoA:amino acid N-acyltransferase",
  "gene_symbol": "BAAT",
  "term_label": "fatty acyl-CoA hydrolase activity",
  "term_id": "GO:0047617",
  "gene": "UniProtKB:Q14032"
}